{
  "gene_name": "Brain-enriched guanylate kinase-associated protein",
  "gene_symbol": "BEGAIN",
  "term_id": "GO:0098817",
  "term_label": "evoked excitatory postsynaptic potential",
  "gene": "UniProtKB:Q9BUH8"
}